cell cycle comprising mitosis without cytokinesis [GO:0033301] (biological process) Relationships: is a type of mitotic cell cycle [GO:0000278] Note: Note that this term should be used for naturally occurring instances of mitosis without cytokinesis, e.g. in the tapetum of flowers and in a number of lower eukaryotes; it should not be used for abnormal events such as may occur in cancers. Subtypes: preblastoderm mitotic cell cycle [GO:0035185], GO:0035186 Definition: A mitotic cell cycle in which mitosis is completed but cytokinesis does not occur, resulting in a cell containing multiple nuclei each with a chromosomal complement of the original ploidy (usually 2N). Sources: GOC:expert_vm, GOC:mah